{
  "term_label": "calcineurin-mediated signaling",
  "gene_name": "Calmodulin-3",
  "term_id": "GO:0097720",
  "gene": "UniProtKB:P0DP25",
  "gene_symbol": "CALM3"
}